{
  "gene_name": "Protein ripply2",
  "gene_symbol": "RIPPLY2",
  "gene": "UniProtKB:Q5TAB7",
  "term_id": "GO:0009880",
  "term_label": "embryonic pattern specification"
}